{
  "gene_symbol": "TMEM178A",
  "term_id": "UNKNOWN:0001",
  "gene": "UniProtKB:Q8NBL3",
  "term_label": "Unknown molecular function",
  "gene_name": "Transmembrane protein 178A"
}